dolichyl-phosphate D-xylosyltransferase activity [GO:0047283] (molecular function) Definition: Catalysis of the reaction: dolichol-phosphate + UDP-D-xylose = dolichyl D-xylosyl phosphate + UDP. Relationships: is a type of UDP-xylosyltransferase activity [GO:0035252] Also known as: UDP-D-xylose:dolichyl-phosphate D-xylosyltransferase activity Sources: EC:2.4.2.32, MetaCyc:2.4.2.32-RXN